negative regulation of ubiquitin protein ligase activity [GO:1904667] (BP) Also known as: down regulation of protein ubiquitination activity, down regulation of ubiquitin ligase activity, down regulation of ubiquitin protein ligase activity, down-regulation of protein ubiquitination activity, down-regulation of ubiquitin ligase activity, down-regulation of ubiquitin protein ligase activity, downregulation of protein ubiquitination activity, downregulation of ubiquitin ligase activity, downregulation of ubiquitin protein ligase activity, negative regulation of protein ubiquitination activity, negative regulation of ubiquitin ligase activity, inhibition of protein ubiquitination activity, inhibition of ubiquitin ligase activity, inhibition of ubiquitin protein ligase activity, negative regulation of APC-Cdc20 complex activity, negative regulation of APC-fizzy related complex activity, down regulation of E3, down-regulation of E3, downregulation of E3, inhibition of E3, negative regulation of APC activity during mitotic cell cycle, negative regulation of APC/C activity during mitotic cell cycle, negative regulation of E3, negative regulation of anaphase-promoting complex activity during mitotic cell cycle, negative regulation of cyclosome activity during mitotic cell cycle, negative regulation of mitotic anaphase-promoting complex activity Relationships: is a type of negative regulation of ubiquitin-protein transferase activity [GO:0051444]; is a type of regulation of ubiquitin protein ligase activity [GO:1904666]; RO_0002212 GO:0061630 References: PMID:26216882 Sources: GOC:TermGenie, GOC:dph, GOC:tb, GO_REF:0000059 Definition: Any process that stops, prevents or reduces the frequency, rate or extent of ubiquitin protein ligase activity.